{
  "gene": "UniProtKB:P15104",
  "term_id": "GO:0005737",
  "gene_name": "Glutamine synthetase",
  "term_label": "cytoplasm",
  "gene_symbol": "GLUL"
}